{
  "term_label": "regulation of transcription by RNA polymerase II",
  "term_id": "GO:0006357",
  "gene": "UniProtKB:Q96N22",
  "gene_name": "Zinc finger protein 681",
  "gene_symbol": "ZNF681"
}